{
  "term_label": "synapse",
  "gene_symbol": "CHRNA6",
  "gene": "UniProtKB:Q15825",
  "term_id": "GO:0045202",
  "gene_name": "Neuronal acetylcholine receptor subunit alpha-6"
}